{
  "gene_name": "Interferon-induced transmembrane protein 3",
  "gene_symbol": "IFITM3",
  "term_label": "plasma membrane",
  "gene": "UniProtKB:Q01628",
  "term_id": "GO:0005886"
}